corneocyte desquamation [GO:0003336] (biological process) Sources: GOC:dph Relationships: is a type of delamination [GO:0060232]; is part of corneocyte development [GO:0003335] Definition: The delamination process that results in the shedding of a corneocyte from the surface of the epidermis. Also known as: epidermal desquamation